{
  "gene_symbol": "MFAP3L",
  "gene": "UniProtKB:O75121",
  "term_id": "GO:0043005",
  "term_label": "neuron projection",
  "gene_name": "Microfibrillar-associated protein 3-like"
}